{
  "term_label": "Unknown biological process",
  "gene": "UniProtKB:A0A6Q8PFD8",
  "gene_symbol": "A0A6Q8PFD8",
  "term_id": "UNKNOWN:0002",
  "gene_name": "Uncharacterized protein"
}